{
  "gene": "UniProtKB:P13500",
  "gene_name": "C-C motif chemokine 2",
  "term_label": "inflammatory response",
  "term_id": "GO:0006954",
  "gene_symbol": "CCL2"
}